regulation of reproductive fruiting body development [GO:0031155] (biological process) Sources: GOC:mah Subtypes: GO:0075268, GO:1902058 Also known as: regulation of fruiting body formation Relationships: is a type of regulation of spore-bearing organ development [GO:0075260]; regulates GO:0030582 Definition: Any process that modulates the frequency, rate or extent of reproductive fruiting body development.